glial cell development [GO:0021782] (biological process) Sources: GOC:cls, GOC:dgh, GOC:dph, GOC:jid, GO_REF:0000021 Definition: The process aimed at the progression of a glial cell over time, from initial commitment of the cell to a specific fate, to the fully functional differentiated cell. Subtypes: astrocyte development [GO:0014002], oligodendrocyte development [GO:0014003], microglia development [GO:0014005], GO:0014044, lateral line nerve glial cell development [GO:0048937], establishment of glial blood-brain barrier [GO:0060857], cardiac glial cell development [GO:0060952] Relationships: is a type of cell development [GO:0048468]; is part of glial cell differentiation [GO:0010001]